cellular response to chlorate [GO:0071246] (biological process) Definition: Any process that results in a change in state or activity of a cell (in terms of movement, secretion, enzyme production, gene expression, etc.) as a result of a chlorate stimulus. Sources: GOC:mah Relationships: is a type of response to chlorate [GO:0010157]; is a type of cellular response to oxygen-containing compound [GO:1901701]